acylglycerol catabolic process [GO:0046464] (biological process) Also known as: acylglycerol breakdown, acylglycerol catabolism, acylglycerol degradation Subtypes: triglyceride catabolic process [GO:0019433], GO:0046340, monoacylglycerol catabolic process [GO:0052651] Relationships: is a type of acylglycerol metabolic process [GO:0006639]; is a type of GO:0046461; is a type of glycerolipid catabolic process [GO:0046503] Definition: The chemical reactions and pathways resulting in the breakdown of acylglycerol, any mono-, di- or triester of glycerol with (one or more) fatty acids. Sources: GOC:ai